positive regulation of fat cell proliferation [GO:0070346] (biological process) Definition: Any process that activates or increases the rate or extent of fat cell proliferation. Subtypes: positive regulation of brown fat cell proliferation [GO:0070349], positive regulation of white fat cell proliferation [GO:0070352] Relationships: is a type of positive regulation of cell population proliferation [GO:0008284]; is a type of regulation of fat cell proliferation [GO:0070344]; positively regulates fat cell proliferation [GO:0070341] Also known as: positive regulation of adipocyte proliferation, positive regulation of adipose cell proliferation, up regulation of fat cell proliferation, up-regulation of fat cell proliferation, upregulation of fat cell proliferation, activation of fat cell proliferation, stimulation of fat cell proliferation Sources: GOC:mah, GOC:sl